chorionic trophoblast cell differentiation [GO:0060718] (biological process) Definition: The process in which relatively unspecialized cells of the ectoplacental cone acquire specialized structural and/or functional features that characterize chorionic trophoblasts. These cells will migrate towards the spongiotrophoblast layer and give rise to syncytiotrophoblasts of the labyrinthine layer. References: PMID:16983341 Sources: CL:0011101, GOC:dph Relationships: is a type of cell differentiation [GO:0030154]; is part of GO:0060717